{
  "gene_symbol": "SLC9C1",
  "term_id": "GO:0098719",
  "gene_name": "Sodium_hydrogen exchanger 10",
  "term_label": "sodium ion import across plasma membrane",
  "gene": "UniProtKB:Q4G0N8"
}